{
  "term_label": "heme binding",
  "gene_name": "ATP-binding cassette sub-family B member 6",
  "gene_symbol": "ABCB6",
  "term_id": "GO:0020037",
  "gene": "UniProtKB:Q9NP58"
}